{
  "gene": "UniProtKB:P52737",
  "term_id": "GO:0005634",
  "term_label": "nucleus",
  "gene_symbol": "ZNF136",
  "gene_name": "Zinc finger protein 136"
}